{
  "gene": "UniProtKB:O95819",
  "gene_name": "Mitogen-activated protein kinase kinase kinase kinase 4",
  "term_label": "MAPK cascade",
  "gene_symbol": "MAP4K4",
  "term_id": "GO:0000165"
}